{
  "gene": "UniProtKB:Q9UBB4",
  "term_id": "GO:0005829",
  "gene_symbol": "ATXN10",
  "gene_name": "Ataxin-10",
  "term_label": "cytosol"
}